{
  "term_id": "UNKNOWN:0002",
  "term_label": "Unknown biological process",
  "gene": "UniProtKB:Q6UWI2",
  "gene_symbol": "PARM1",
  "gene_name": "Prostate androgen-regulated mucin-like protein 1"
}